{
  "term_id": "GO:0000981",
  "gene": "UniProtKB:Q9HB58",
  "gene_name": "Sp110 nuclear body protein",
  "term_label": "DNA-binding transcription factor activity, RNA polymerase II-specific",
  "gene_symbol": "SP110"
}